{
  "gene": "UniProtKB:P26196",
  "gene_symbol": "DDX6",
  "gene_name": "Probable ATP-dependent RNA helicase DDX6",
  "term_id": "GO:0017148",
  "term_label": "negative regulation of translation"
}